{
  "gene_symbol": "POSTN",
  "gene_name": "Periostin",
  "term_label": "cell adhesion molecule binding",
  "gene": "UniProtKB:Q15063",
  "term_id": "GO:0050839"
}